{
  "gene_symbol": "EPHA3",
  "gene": "UniProtKB:P29320",
  "term_label": "dendrite",
  "term_id": "GO:0030425",
  "gene_name": "Ephrin type-A receptor 3"
}